{
  "gene": "UniProtKB:P20594",
  "term_id": "GO:0017046",
  "gene_symbol": "NPR2",
  "gene_name": "Atrial natriuretic peptide receptor 2",
  "term_label": "peptide hormone binding"
}